immune complex clearance by monocytes and macrophages [GO:0002436] (biological process) Sources: GOC:add, ISBN:0781735149 Relationships: is a type of immune complex clearance [GO:0002434] Regulation: regulated by regulation of immune complex clearance by monocytes and macrophages [GO:0090264]; positively regulated by positive regulation of immune complex clearance by monocytes and macrophages [GO:0090265] Definition: The process of immune complex clearance by monocytes or macrophages.